{
  "gene_name": "RNA-binding motif protein, X chromosome",
  "term_label": "spliceosomal complex",
  "term_id": "GO:0005681",
  "gene_symbol": "RBMX",
  "gene": "UniProtKB:P38159"
}